glycosphingolipid binding [GO:0043208] (molecular function) Subtypes: ganglioside binding [GO:0035594] Sources: GOC:jl Relationships: is_a sphingolipid binding [GO:0046625]; is a type of glycolipid binding [GO:0051861] Definition: Binding to glycosphingolipid, a compound with residues of sphingoid and at least one monosaccharide.